{
  "gene_symbol": "SLC17A8",
  "term_label": "neurotransmitter loading into synaptic vesicle",
  "term_id": "GO:0098700",
  "gene_name": "Vesicular glutamate transporter 3",
  "gene": "UniProtKB:Q8NDX2"
}